postsynaptic early endosome membrane [GO:0098896] (CC) Sources: GOC:pz Definition: The lipid bilayer surrounding a postsynaptic early endosome. Relationships: is a type of early endosome membrane [GO:0031901]; is a type of postsynaptic endosome membrane [GO:0098895]; is part of postsynaptic early endosome [GO:0098842]